{
  "gene_symbol": "NCBP2",
  "term_label": "RNA cap binding",
  "term_id": "GO:0000339",
  "gene": "UniProtKB:P52298",
  "gene_name": "Nuclear cap-binding protein subunit 2"
}